{
  "gene_name": "Dynein assembly factor with WDR repeat domains 1",
  "term_id": "GO:0019005",
  "gene": "UniProtKB:Q8N136",
  "gene_symbol": "DAW1",
  "term_label": "SCF ubiquitin ligase complex"
}